{
  "gene": "UniProtKB:P33151",
  "gene_symbol": "CDH5",
  "term_id": "GO:0034332",
  "term_label": "adherens junction organization",
  "gene_name": "Cadherin-5"
}